{
  "gene_symbol": "NEGR1",
  "gene_name": "Neuronal growth regulator 1",
  "gene": "UniProtKB:Q7Z3B1",
  "term_id": "GO:0051963",
  "term_label": "regulation of synapse assembly"
}